{
  "gene_name": "RNA-binding protein 26",
  "gene_symbol": "RBM26",
  "term_label": "nucleus",
  "gene": "UniProtKB:Q5T8P6",
  "term_id": "GO:0005634"
}